{
  "term_id": "GO:0006606",
  "gene_name": "Nuclear pore-associated protein 1",
  "term_label": "protein import into nucleus",
  "gene_symbol": "NPAP1",
  "gene": "UniProtKB:Q9NZP6"
}